telophase [GO:0051326] (biological process) Relationships: is a type of cell cycle phase [GO:0022403]; is part of M phase [GO:0000279] Subtypes: mitotic telophase [GO:0000093], meiotic telophase I [GO:0007134], meiotic telophase II [GO:0007139] Note: note that this term should not be used for direct annotation. if you are trying to make an annotation to x phase, it is likely that the correct annotation is 'regulation of x/y phase transition' or to a process which occurs during the reported phase (i.e mitotic DNA replication for mitotic s-phase). to capture the phase when a specific location or process is observed, the phase term can be used in an annotation extension (PMID:24885854) applied to a cellular component term (with the relation exists_during) or a biological process term (with the relation happens_during). Definition: The cell cycle phase which follows anaphase during M phase of mitosis and meiosis and during which the chromosomes arrive at the poles of the cell and the division of the cytoplasm starts. Sources: GOC:mtg_cell_cycle